{
  "gene": "UniProtKB:Q15306",
  "term_label": "nucleus",
  "gene_symbol": "IRF4",
  "term_id": "GO:0005634",
  "gene_name": "Interferon regulatory factor 4"
}